{
  "term_id": "GO:0015141",
  "gene": "UniProtKB:Q8WWT9",
  "gene_name": "Na(+)_dicarboxylate cotransporter 3",
  "gene_symbol": "SLC13A3",
  "term_label": "succinate transmembrane transporter activity"
}